{
  "term_id": "UNKNOWN:0003",
  "gene_symbol": "TTC9B",
  "gene_name": "Tetratricopeptide repeat protein 9B",
  "term_label": "Unknown cellular component",
  "gene": "UniProtKB:Q8N6N2"
}